dol-P-Man:Man(8)GlcNAc(2)-PP-Dol alpha-1,2-mannosyltransferase activity [GO:0052918] (molecular function) Definition: Catalysis of the reaction: an alpha-D-Man-(1->2)-alpha-D-Man-(1->2)-alpha-D-Man-(1->3)-[alpha-D-Man-(1->2)-alpha-D-Man-(1->3)-[alpha-D-Man-(1->6)]-alpha-D-Man-(1->6)]-beta-D-Man-(1->4)-beta-D-GlcNAc-(1->4)-alpha-D-GlcNAc-diphospho-di-trans,poly-cis-dolichol + a di-trans,poly-cis-dolichyl beta-D-mannosyl phosphate = an alpha-D-Man-(1->2)-alpha-D-Man-(1->2)-alpha-D-Man-(1->3)-[alpha-D-Man-(1->2)-alpha-D-Man-(1->3)-[alpha-D-Man-(1->2)-alpha-D-Man-(1->6)]-alpha-D-Man-(1->6)]-beta-D-Man-(1->4)-beta-D-GlcNAc-(1->4)-alpha-D-GlcNAc-diphospho-di-trans,poly-cis-dolichol + a di-trans,poly-cis-dolichyl phosphate + H+. Sources: RHEA:29539 Relationships: is a type of alpha-1,2-mannosyltransferase activity [GO:0000026]; is a type of GO:0120562